{
  "term_label": "negative regulation of double-strand break repair via homologous recombination",
  "gene_name": "RecQ-mediated genome instability protein 2",
  "gene": "UniProtKB:Q96E14",
  "gene_symbol": "RMI2",
  "term_id": "GO:2000042"
}